{
  "term_id": "UNKNOWN:0001",
  "gene_symbol": "CRB1",
  "gene_name": "Protein crumbs homolog 1",
  "gene": "UniProtKB:P82279",
  "term_label": "Unknown molecular function"
}